{
  "gene_symbol": "CLEC2D",
  "term_label": "plasma membrane",
  "gene_name": "C-type lectin domain family 2 member D",
  "term_id": "GO:0005886",
  "gene": "UniProtKB:Q9UHP7"
}